choline dehydrogenase activity [GO:0008812] (molecular function) Subtypes: choline monooxygenase (NADP+) activity [GO:0102280] Definition: Catalysis of the reaction: A + choline = AH(2) + betaine aldehyde. Also known as: choline oxidase activity, choline-cytochrome c reductase activity, choline:(acceptor) 1-oxidoreductase activity, choline:(acceptor) oxidoreductase activity, choline:acceptor 1-oxidoreductase activity Relationships: is a type of oxidoreductase activity, acting on CH-OH group of donors [GO:0016614] Sources: EC:1.1.99.1, RHEA:17433